haptoglobin binding [GO:0031720] (molecular function) Definition: Binding to a haptoglobin, any alpha2 globulin of blood plasma that can combine with free oxyhemoglobin to form a stable complex. Sources: GOC:mah, ISBN:0198506732 Relationships: is_a protein binding [GO:0005515]